{
  "term_label": "Unknown biological process",
  "gene_symbol": "ISM2",
  "gene": "UniProtKB:Q6H9L7",
  "gene_name": "Isthmin-2",
  "term_id": "UNKNOWN:0002"
}